integrin alpha10-beta1 complex [GO:0034680] (cellular component) Definition: An integrin complex that comprises one alpha10 subunit and one beta1 subunit. References: PMID:12297042 Also known as: alpha10-beta1 integrin complex, ITGA10-ITGB1 complex Relationships: is a type of integrin complex [GO:0008305]